nuclear transport [GO:0051169] (biological process) Also known as: nucleus transport Relationships: is a type of intracellular transport [GO:0046907] Sources: GOC:ai Definition: The directed movement of substances into, out of, or within the nucleus. Subtypes: nucleocytoplasmic transport [GO:0006913]